{
  "term_label": "delayed rectifier potassium channel activity",
  "term_id": "GO:0005251",
  "gene": "UniProtKB:Q09470",
  "gene_name": "Potassium voltage-gated channel subfamily A member 1",
  "gene_symbol": "KCNA1"
}